{
  "term_id": "GO:0003743",
  "gene_name": "Eukaryotic translation initiation factor 2 subunit 3",
  "gene_symbol": "EIF2S3",
  "term_label": "translation initiation factor activity",
  "gene": "UniProtKB:P41091"
}